peroxiredoxin activity [GO:0051920] (molecular function) Subtypes: NADH-dependent peroxiredoxin activity [GO:0102039], thioredoxin-dependent peroxiredoxin activity [GO:0140824] Sources: RHEA:10008 Also known as: PRDX activity, Prx activity Relationships: is_a peroxidase activity [GO:0004601] Definition: Catalysis of the reaction: [protein]-dithol + ROOH = [protein]-disulfide + H2O + ROH. Note: Includes redox chemistry as part of the catalytic reaction (2 R'-SH = R'-S-S-R'), where R' refers to peroxiredoxin itself). Not to be confused with GO:0004601 (peroxidase activity, EC:1.11.1.7), which has a different reaction mechanism.